{
  "term_id": "GO:0005615",
  "gene_name": "Gastrin-releasing peptide",
  "term_label": "extracellular space",
  "gene": "UniProtKB:P07492",
  "gene_symbol": "GRP"
}